{
  "gene_symbol": "LINC02881",
  "term_id": "UNKNOWN:0002",
  "gene": "UniProtKB:B7Z368",
  "term_label": "Unknown biological process",
  "gene_name": "Uncharacterized protein encoded by LINC02881"
}